killing by virus of host cell during superinfection exclusion [GO:0039634] (biological process) References: PMID:22398285 Sources: GOC:bf, GOC:bm, GOC:jl Relationships: is a type of symbiont-mediated killing of host cell [GO:0001907]; is a type of response to virus [GO:0009615] Also known as: killing by virus of host cells during superinfection exclusion, killing by virus of host cells involved in superinfection exclusion, Rex exclusion Definition: The viral-killing of a host cell by a pre-existing virus in response to a subsequent infection of the host cell by second virus.